mitochondrial small ribosomal subunit [GO:0005763] (cellular component) Sources: GOC:mcc Relationships: is a type of GO:0000314; is_a GO:0098798; BFO_0000050 mitochondrial ribosome [GO:0005761] Definition: The smaller of the two subunits of a mitochondrial ribosome. Also known as: mitochondrial ribosomal SSU complex, mitochondrial ribosomal small subunit complex, 28S ribosomal subunit, mitochondrial